cell fate commitment involved in pattern specification [GO:0060581] (biological process) Subtypes: GO:0035052, dorsal vessel heart proper cell fate commitment [GO:0035053], GO:0060579, GO:0060898 Relationships: is a type of GO:0045165; is part of pattern specification process [GO:0007389] Sources: GOC:dph Definition: The commitment of cells to specific cell fates and their capacity to differentiate into particular kinds of cells within a field of cells that will exhibit a certain pattern of differentiation. Positional information is established through protein signals that emanate from a localized source within a developmental field resulting in specification of a cell type. Those signals are then interpreted in a cell-autonomous manner resulting in the determination of the cell type.